{
  "gene": "UniProtKB:Q7Z3T8",
  "term_id": "GO:0006622",
  "gene_name": "Zinc finger FYVE domain-containing protein 16",
  "term_label": "protein targeting to lysosome",
  "gene_symbol": "ZFYVE16"
}